GMP metabolic process [GO:0046037] (biological process) Subtypes: GMP biosynthetic process [GO:0006177], GMP catabolic process [GO:0046038] Relationships: is a type of purine ribonucleotide metabolic process [GO:0009150]; is a type of purine ribonucleoside monophosphate metabolic process [GO:0009167] Sources: GOC:go_curators Definition: The chemical reactions and pathways involving GMP, guanosine monophosphate. Also known as: GMP metabolism